{
  "gene": "UniProtKB:Q9BVA1",
  "term_label": "GTP binding",
  "gene_name": "Tubulin beta-2B chain",
  "term_id": "GO:0005525",
  "gene_symbol": "TUBB2B"
}